{
  "gene_symbol": "CCL8",
  "gene": "UniProtKB:P80075",
  "term_label": "antimicrobial humoral immune response mediated by antimicrobial peptide",
  "term_id": "GO:0061844",
  "gene_name": "C-C motif chemokine 8"
}